{
  "term_label": "Unknown molecular function",
  "gene": "UniProtKB:A0JNW5",
  "term_id": "UNKNOWN:0001",
  "gene_symbol": "BLTP3B",
  "gene_name": "Bridge-like lipid transfer protein family member 3B"
}